{
  "term_label": "cell surface receptor signaling pathway",
  "term_id": "GO:0007166",
  "gene_name": "T cell receptor beta variable 6-5",
  "gene": "UniProtKB:A0A0K0K1A5",
  "gene_symbol": "TRBV6-5"
}